{
  "term_id": "UNKNOWN:0003",
  "gene_symbol": "RLBP1",
  "gene_name": "Retinaldehyde-binding protein 1",
  "gene": "UniProtKB:P12271",
  "term_label": "Unknown cellular component"
}